{
  "gene": "UniProtKB:Q9NRX6",
  "gene_name": "Protein kish-B",
  "term_label": "Unknown biological process",
  "gene_symbol": "TMEM167B",
  "term_id": "UNKNOWN:0002"
}